{
  "gene_name": "Pannexin-3",
  "gene_symbol": "PANX3",
  "term_id": "GO:0007267",
  "gene": "UniProtKB:Q96QZ0",
  "term_label": "cell-cell signaling"
}